{
  "gene": "UniProtKB:P17014",
  "gene_name": "Zinc finger protein 12",
  "term_label": "DNA-binding transcription factor activity, RNA polymerase II-specific",
  "term_id": "GO:0000981",
  "gene_symbol": "ZNF12"
}